{
  "term_label": "nucleus",
  "gene_name": "Zinc finger protein 641",
  "term_id": "GO:0005634",
  "gene_symbol": "ZNF641",
  "gene": "UniProtKB:Q96N77"
}